isopeptide cross-linking [GO:0018262] (biological process) Relationships: is a type of peptide cross-linking [GO:0018149] Sources: GOC:jsg Definition: The formation of a covalent cross-link between or within peptide chains, where either the amino group or the carboxyl group, or both, are not attached to the alpha carbon. Subtypes: GO:0018153